{
  "gene": "UniProtKB:Q9P281",
  "gene_name": "BAH and coiled-coil domain-containing protein 1",
  "term_label": "Unknown biological process",
  "term_id": "UNKNOWN:0002",
  "gene_symbol": "BAHCC1"
}